{
  "term_label": "Unknown cellular component",
  "term_id": "UNKNOWN:0003",
  "gene": "UniProtKB:Q7Z736",
  "gene_symbol": "PLEKHH3",
  "gene_name": "Pleckstrin homology domain-containing family H member 3"
}